negative regulation of follicle-stimulating hormone secretion [GO:0046882] (biological process) Also known as: down regulation of follicle-stimulating hormone secretion, down-regulation of follicle-stimulating hormone secretion, downregulation of follicle-stimulating hormone secretion, negative regulation of follicle stimulating hormone secretion, inhibition of follicle-stimulating hormone secretion Relationships: is a type of negative regulation of gonadotropin secretion [GO:0032277]; is a type of regulation of follicle-stimulating hormone secretion [GO:0046880]; negatively regulates GO:0046884 Sources: GOC:ai Definition: Any process that stops, prevents, or reduces the frequency, rate or extent of the regulated release of follicle-stimulating hormone.